{
  "gene_name": "Neuropeptide S",
  "term_id": "GO:0051968",
  "gene": "UniProtKB:P0C0P6",
  "term_label": "positive regulation of synaptic transmission, glutamatergic",
  "gene_symbol": "NPS"
}